{
  "gene": "UniProtKB:Q9C0D2",
  "term_label": "centriole",
  "gene_symbol": "CEP295",
  "term_id": "GO:0005814",
  "gene_name": "Centrosomal protein of 295 kDa"
}